xyloglucan-specific endo-beta-1,4-glucanase activity [GO:0033946] (molecular function) Sources: EC:3.2.1.151 Definition: Catalysis of the reaction: xyloglucan + H2O = xyloglucan oligosaccharides. This reaction is the endohydrolysis of (1->4)-beta-D-glucosidic linkages in xyloglucan. Also known as: 1,4-beta-D-glucan glucanohydrolase activity, XEG, XH, [(1->6)-beta-D-xylo]-(1->4)-beta-D-glucan glucanohydrolase activity, xyloglucan endo-beta-1,4-glucanase activity, xyloglucanase activity, xyloglucanendohydrolase activity Relationships: is a type of beta-glucanase activity [GO:0052736] Regulation: negatively regulated by xyloglucan-specific endo-beta-1,4-glucanase inhibitor activity [GO:0140594]